{
  "gene_name": "Amine oxidase [flavin-containing] A",
  "gene_symbol": "MAOA",
  "term_label": "serotonin metabolic process",
  "gene": "UniProtKB:P21397",
  "term_id": "GO:0042428"
}